prosthetic group binding [GO:0051192] (molecular function) Definition: Binding to a prosthetic group, the non-amino acid portion of certain protein molecules. Prosthetic groups may be inorganic or organic and are usually required for the biological activity of the protein. Sources: GOC:ai, GOC:vw Subtypes: ACP phosphopantetheine attachment site binding [GO:0044620] Relationships: is_a binding [GO:0005488]